pulmonary valve formation [GO:0003193] (biological process) Sources: GOC:mtg_heart Definition: The developmental process pertaining to the initial formation of the pulmonary valve from unspecified parts. This process begins with the specific processes that contribute to the appearance of the discrete structure and ends when the structural rudiment is recognizable. Relationships: is_a heart valve formation [GO:0003188]; is part of GO:0003184